{
  "gene": "UniProtKB:Q0VD86",
  "term_label": "cyclin binding",
  "term_id": "GO:0030332",
  "gene_name": "Protein INCA1",
  "gene_symbol": "INCA1"
}